{
  "gene_symbol": "ERCC1",
  "gene_name": "DNA excision repair protein ERCC-1",
  "term_id": "GO:0070522",
  "term_label": "ERCC4-ERCC1 complex",
  "gene": "UniProtKB:P07992"
}